{
  "gene_symbol": "C1QTNF3",
  "gene": "UniProtKB:Q9BXJ4",
  "term_label": "extracellular space",
  "term_id": "GO:0005615",
  "gene_name": "Complement C1q tumor necrosis factor-related protein 3"
}